{
  "gene_symbol": "DNAJB11",
  "term_label": "endoplasmic reticulum",
  "gene_name": "DnaJ homolog subfamily B member 11",
  "term_id": "GO:0005783",
  "gene": "UniProtKB:Q9UBS4"
}